regulation of maintenance of mitotic sister chromatid cohesion [GO:0034182] (biological process) Sources: GOC:mah, GOC:vw Relationships: is a type of GO:0034091; regulates maintenance of mitotic sister chromatid cohesion [GO:0034088] Definition: Any process that modulates the extent to which the association between sister chromatids of a replicated chromosome is maintained during a mitotic cell cycle. Subtypes: negative regulation of maintenance of mitotic sister chromatid cohesion [GO:0034183], positive regulation of maintenance of mitotic sister chromatid cohesion [GO:0034184], regulation of maintenance of mitotic sister chromatid cohesion, telomeric [GO:1904907], regulation of maintenance of mitotic sister chromatid cohesion, arms [GO:2000715], regulation of maintenance of mitotic sister chromatid cohesion, centromeric [GO:2000718]